{
  "term_label": "Unknown biological process",
  "gene": "UniProtKB:O95297",
  "term_id": "UNKNOWN:0002",
  "gene_name": "Myelin protein zero-like protein 1",
  "gene_symbol": "MPZL1"
}